{
  "gene_symbol": "CFP",
  "term_label": "Unknown cellular component",
  "gene_name": "Properdin",
  "gene": "UniProtKB:P27918",
  "term_id": "UNKNOWN:0003"
}